{
  "gene": "UniProtKB:P09131",
  "gene_name": "P3 protein",
  "term_label": "bile acid and bile salt transport",
  "term_id": "GO:0015721",
  "gene_symbol": "SLC10A3"
}